{
  "gene": "UniProtKB:O75448",
  "gene_name": "Mediator of RNA polymerase II transcription subunit 24",
  "term_id": "GO:0060261",
  "term_label": "positive regulation of transcription initiation by RNA polymerase II",
  "gene_symbol": "MED24"
}